{
  "gene_symbol": "ASPG",
  "gene_name": "60 kDa lysophospholipase",
  "gene": "UniProtKB:Q86U10",
  "term_id": "GO:0004067",
  "term_label": "asparaginase activity"
}